{
  "gene_name": "Ornithine decarboxylase",
  "term_id": "GO:0004586",
  "term_label": "ornithine decarboxylase activity",
  "gene": "UniProtKB:P11926",
  "gene_symbol": "ODC1"
}